negative regulation of mRNA processing [GO:0050686] (biological process) Sources: GOC:ai Relationships: is a type of regulation of mRNA processing [GO:0050684]; is a type of negative regulation of mRNA metabolic process [GO:1903312]; negatively regulates mRNA processing [GO:0006397] Definition: Any process that stops, prevents, or reduces the frequency, rate or extent of mRNA processing. Subtypes: negative regulation of mRNA 3'-end processing [GO:0031441], negative regulation of mRNA splicing, via spliceosome [GO:0048025] Also known as: down regulation of mRNA processing, down-regulation of mRNA processing, downregulation of mRNA processing, inhibition of mRNA processing